{
  "gene_name": "Olfactory receptor 4N4",
  "gene_symbol": "OR4N4",
  "term_id": "GO:0005886",
  "gene": "UniProtKB:Q8N0Y3",
  "term_label": "plasma membrane"
}